alpha3-beta1 integrin-CD63 complex [GO:0071081] (cellular component) Also known as: ITGA3-ITGB1-CD63 complex References: PMID:7629079 Definition: A protein complex that consists of an alpha3-beta1 integrin complex bound to the tetraspanin CD63. Relationships: is a type of plasma membrane protein complex [GO:0098797]